{
  "term_id": "GO:0000149",
  "gene_symbol": "ANKRD27",
  "gene": "UniProtKB:Q96NW4",
  "gene_name": "Ankyrin repeat domain-containing protein 27",
  "term_label": "SNARE binding"
}